{
  "gene_symbol": "PFDN2",
  "term_label": "protein folding",
  "gene_name": "Prefoldin subunit 2",
  "gene": "UniProtKB:Q9UHV9",
  "term_id": "GO:0006457"
}